rRNA transport [GO:0051029] (biological process) Sources: GOC:ai Definition: The directed movement of rRNA, ribosomal ribonucleic acid, into, out of or within a cell, or between cells, by means of some agent such as a transporter or pore. Subtypes: mitochondrial rRNA export from mitochondrion [GO:0019090], rRNA import into mitochondrion [GO:0035928] Relationships: is a type of GO:0050658